recombinational repair [GO:0000725] (biological process) Sources: GOC:elh Definition: A DNA repair process that involves the exchange, reciprocal or nonreciprocal, of genetic material between the broken DNA molecule and a homologous DNA region. Subtypes: GO:0000724, GO:0036298, mitochondrial double-strand break repair via homologous recombination [GO:0097552], GO:1990396 Relationships: is a type of DNA repair [GO:0006281]; is a type of GO:0006310